{
  "gene_name": "Outer dynein arm-docking complex subunit 4",
  "term_id": "GO:0005737",
  "term_label": "cytoplasm",
  "gene_symbol": "ODAD4",
  "gene": "UniProtKB:Q96NG3"
}